{
  "gene": "UniProtKB:P11150",
  "gene_name": "Hepatic triacylglycerol lipase",
  "gene_symbol": "LIPC",
  "term_label": "extracellular space",
  "term_id": "GO:0005615"
}